hermaphrodite somatic sex determination [GO:0042001] (biological process) Subtypes: GO:0042003, feminization of hermaphrodite soma [GO:0042004] Definition: The determination of sex and sexual phenotypes in a hermaphroditic organism's soma. An example of this is found in Caenorhabditis elegans. Relationships: is a type of somatic sex determination [GO:0018993] Sources: GOC:ems